Cul5-RING ubiquitin ligase complex [GO:0031466] (cellular component) Definition: A ubiquitin ligase complex in which a cullin from the Cul5 subfamily and a RING domain protein form the catalytic core; substrate specificity is conferred by an elongin-BC adaptor and a SOCS/BC box protein. References: PMID:15571813, PMID:15688063 Also known as: EC2S complex, CDL5 complex, CRL5 complex, cullin-RING ligase 5, SCF5 complex Relationships: is a type of cullin-RING ubiquitin ligase complex [GO:0031461]